{
  "term_label": "Unknown cellular component",
  "gene": "UniProtKB:Q8NA61",
  "term_id": "UNKNOWN:0003",
  "gene_name": "Protein chibby homolog 2",
  "gene_symbol": "CBY2"
}